{
  "gene_symbol": "SHANK1",
  "term_label": "postsynaptic density",
  "term_id": "GO:0014069",
  "gene": "UniProtKB:Q9Y566",
  "gene_name": "SH3 and multiple ankyrin repeat domains protein 1"
}